{
  "term_id": "GO:0006612",
  "gene_symbol": "NACAD",
  "gene": "UniProtKB:O15069",
  "term_label": "protein targeting to membrane",
  "gene_name": "NAC-alpha domain-containing protein 1"
}